{
  "term_id": "GO:0043161",
  "term_label": "proteasome-mediated ubiquitin-dependent protein catabolic process",
  "gene_name": "BTB_POZ domain-containing protein KCTD5",
  "gene_symbol": "KCTD5",
  "gene": "UniProtKB:Q9NXV2"
}